pre-T cell receptor complex [GO:0043384] (cellular component) Also known as: pre-T lymphocyte receptor complex, pre-T-cell receptor complex, pre-T-lymphocyte receptor complex, pre-TCR complex References: PMID:12220932 Sources: ISBN:0781735149 Definition: A receptor complex found on immature T cells consisting of a T cell receptor beta chain and the pre-TCR-alpha chain, along with additional signaling components including CD3 family members and additional signaling proteins. Relationships: is a type of GO:0098802